{
  "gene_symbol": "FOXE1",
  "gene": "UniProtKB:O00358",
  "term_label": "cell differentiation",
  "term_id": "GO:0030154",
  "gene_name": "Forkhead box protein E1"
}